{
  "term_id": "GO:0001817",
  "gene_symbol": "BTNL8",
  "gene_name": "Butyrophilin-like protein 8",
  "gene": "UniProtKB:Q6UX41",
  "term_label": "regulation of cytokine production"
}